{
  "term_id": "GO:0005737",
  "gene_name": "E3 ubiquitin-protein ligase MARCHF1",
  "gene_symbol": "MARCHF1",
  "gene": "UniProtKB:Q8TCQ1",
  "term_label": "cytoplasm"
}